{
  "gene_name": "Tyrosine-protein kinase Fyn",
  "term_id": "GO:0004715",
  "term_label": "non-membrane spanning protein tyrosine kinase activity",
  "gene_symbol": "FYN",
  "gene": "UniProtKB:P06241"
}